{
  "term_label": "positive regulation of cytosolic calcium ion concentration",
  "gene_symbol": "TBXA2R",
  "gene_name": "Thromboxane A2 receptor",
  "term_id": "GO:0007204",
  "gene": "UniProtKB:P21731"
}